beak development [GO:0071728] (biological process) Relationships: is a type of GO:0048856 Sources: GOC:lp, ISBN:0702008729 Definition: The progression of the beak over time from its initial formation until its mature state. The avian beak is an external anatomical structure, in the head region, that is adapted for feeding self and young, catching prey, probing, etc. It encompasses, but is not restricted to, the maxilla, mandible, maxillary rhamphotheca, mandibular rhamphotheca, nostril, nasal fossa, nasal bones, egg tooth and rictus.